{
  "gene_name": "Zinc finger protein 226",
  "term_label": "nucleus",
  "gene": "UniProtKB:Q9NYT6",
  "term_id": "GO:0005634",
  "gene_symbol": "ZNF226"
}